{
  "term_label": "endosome",
  "term_id": "GO:0005768",
  "gene_symbol": "RAB33B",
  "gene": "UniProtKB:Q9H082",
  "gene_name": "Ras-related protein Rab-33B"
}